invasive growth in response to pheromone [GO:0045311] (biological process) Sources: GOC:ai, GOC:dph, GOC:mcc Relationships: is a type of invasive filamentous growth [GO:0036267]; is part of response to pheromone [GO:0019236] Definition: The growth of colonies in filamentous chains of cells as a result of a pheromone stimulus.